{
  "term_label": "basolateral plasma membrane",
  "term_id": "GO:0016323",
  "gene_symbol": "DLG3",
  "gene": "UniProtKB:Q92796",
  "gene_name": "Disks large homolog 3"
}